{
  "gene_name": "GATOR complex protein WDR24",
  "term_label": "positive regulation of macroautophagy",
  "term_id": "GO:0016239",
  "gene": "UniProtKB:Q96S15",
  "gene_symbol": "WDR24"
}